platelet activating factor biosynthetic process [GO:0006663] (biological process) Sources: ISBN:0198547684 Relationships: is a type of GO:0008611; is a type of GO:0046469; is a type of glycerophospholipid biosynthetic process [GO:0046474] Definition: The chemical reactions and pathways resulting in the formation of platelet activating factor, 1-O-alkyl-2-acetyl-sn-glycerol 3-phosphocholine, where alkyl = hexadecyl or octadecyl. Platelet activating factor is an inflammatory mediator released from a variety of cells in response to various stimuli. Also known as: PAF biosynthesis, PAF biosynthetic process, platelet activating factor anabolism, platelet activating factor biosynthesis, platelet activating factor formation, platelet activating factor synthesis